{
  "gene_name": "Glycine dehydrogenase (decarboxylating), mitochondrial",
  "gene_symbol": "GLDC",
  "term_id": "GO:0004375",
  "gene": "UniProtKB:P23378",
  "term_label": "glycine dehydrogenase (decarboxylating) activity"
}